microtubule depolymerization [GO:0007019] (biological process) Definition: The removal of tubulin heterodimers from one or both ends of a microtubule. Sources: ISBN:0815316194 Also known as: microtubule disassembly, microtubule shortening, microtubule catastrophe, microtubule depolymerization during nuclear congression Subtypes: cytoplasmic microtubule depolymerization [GO:0010938], minus-end specific microtubule depolymerization [GO:0036078], GO:0060172, plus-end specific microtubule depolymerization [GO:0070462], mitotic spindle microtubule depolymerization [GO:1990755] Regulation: negatively regulated by negative regulation of microtubule depolymerization [GO:0007026]; RO_0002211 by regulation of microtubule depolymerization [GO:0031114]; positively regulated by positive regulation of microtubule depolymerization [GO:0031117] Relationships: is a type of GO:0031109; is a type of protein depolymerization [GO:0051261]; is a type of supramolecular fiber organization [GO:0097435]